RNA topoisomerase activity [GO:0140226] (molecular function) References: PMID:23912945, PMID:27257063 Sources: GOC:lnp Definition: Catalysis of the transient cleavage and passage of individual RNA strands or double helices through one another, resulting a topological transformation in RNA. Relationships: is a type of GO:0120545; is a type of catalytic activity, acting on RNA [GO:0140098]